{
  "gene_name": "Kelch-like protein 24",
  "gene": "UniProtKB:Q6TFL4",
  "gene_symbol": "KLHL24",
  "term_label": "Cul3-RING ubiquitin ligase complex",
  "term_id": "GO:0031463"
}